reorganization of cellular membranes to establish viral sites of replication [GO:0140754] (BP) Definition: A process in intracellular membranes are reorganized by viral proteins that perturb membrane integrity and can cause an extensive rearrangement of cellular membranes, forming membranous webs, which are thought to be the site of replication or certain viruses, for example the HPV virus. References: PMID:19376974 Relationships: is a type of symbiont-mediated perturbation of host membrane [GO:0141171]